{
  "term_id": "UNKNOWN:0001",
  "gene": "UniProtKB:Q6UWN0",
  "term_label": "Unknown molecular function",
  "gene_name": "Ly6_PLAUR domain-containing protein 4",
  "gene_symbol": "LYPD4"
}